{
  "term_id": "UNKNOWN:0001",
  "gene_symbol": "EGFEM1P",
  "gene_name": "Putative EGF-like and EMI domain-containing protein 1",
  "term_label": "Unknown molecular function",
  "gene": "UniProtKB:Q0D2K5"
}